{
  "term_id": "UNKNOWN:0002",
  "gene_symbol": "ITPRIPL1",
  "term_label": "Unknown biological process",
  "gene": "UniProtKB:Q6GPH6",
  "gene_name": "Inositol 1,4,5-trisphosphate receptor-interacting protein-like 1"
}